{
  "gene": "UniProtKB:Q9BYQ0",
  "term_label": "Unknown molecular function",
  "gene_symbol": "KRTAP9-8",
  "gene_name": "Keratin-associated protein 9-8",
  "term_id": "UNKNOWN:0001"
}